{
  "term_id": "GO:0005615",
  "gene_symbol": "NTF3",
  "gene": "UniProtKB:P20783",
  "gene_name": "Neurotrophin-3",
  "term_label": "extracellular space"
}